{
  "gene_symbol": "C19orf44",
  "gene": "UniProtKB:Q9H6X5",
  "term_id": "UNKNOWN:0002",
  "gene_name": "Uncharacterized protein C19orf44",
  "term_label": "Unknown biological process"
}